ceramide biosynthetic process [GO:0046513] (biological process) Relationships: is a type of GO:0006672; is a type of sphingolipid biosynthetic process [GO:0030148]; is a type of amide biosynthetic process [GO:0043604] Regulation: negatively regulated by GO:1900060; RO_0002211 by regulation of ceramide biosynthetic process [GO:2000303]; positively regulated by GO:2000304 Also known as: ceramide anabolism, ceramide biosynthesis, ceramide formation, ceramide synthesis Subtypes: lactosylceramide biosynthetic process [GO:0001572], ganglioside biosynthetic process [GO:0001574], glucosylceramide biosynthetic process [GO:0006679], GO:0006682, GO:0106342, GO:1990387 Definition: The chemical reactions and pathways resulting in the formation of ceramides, any N-acylated sphingoid. Sources: GOC:ai